adhesion of symbiont appressorium to host [GO:0075003] (biological process) Definition: The attachment of an appressorium of the symbiont to its host via adhesion molecules. The host is defined as the larger of the organisms involved in a symbiotic interaction. Sources: GOC:pamgo_curators Relationships: is a type of adhesion of symbiont infection structure to host [GO:0075001]; is part of appressorium formation [GO:0075016] Also known as: adhesion of symbiont appressorium to host during symbiotic interaction Note: Note that this term should not be used to annotate gene products of the host. It should only be used to annotate those gene products from the symbiont involved in this process.